{
  "gene_symbol": "NUTM2F",
  "term_id": "UNKNOWN:0001",
  "gene": "UniProtKB:A1L443",
  "term_label": "Unknown molecular function",
  "gene_name": "NUT family member 2F"
}